regulation of mannan catabolic process [GO:2000994] (biological process) Relationships: is a type of GO:2000966; regulates GO:0046355 Subtypes: negative regulation of mannan catabolic process [GO:2000995], positive regulation of mannan catabolic process [GO:2000996] Sources: GOC:mengo_curators Definition: Any process that modulates the frequency, rate or extent of mannan catabolic process. Also known as: regulation of mannan breakdown, regulation of mannan catabolism, regulation of mannan degradation